{
  "gene_name": "1-phosphatidylinositol 4,5-bisphosphate phosphodiesterase eta-1",
  "term_label": "phosphatidylinositol metabolic process",
  "gene": "UniProtKB:Q4KWH8",
  "term_id": "GO:0046488",
  "gene_symbol": "PLCH1"
}